{
  "gene": "UniProtKB:Q6IQ32",
  "term_id": "UNKNOWN:0001",
  "term_label": "Unknown molecular function",
  "gene_name": "Activity-dependent neuroprotector homeobox protein 2",
  "gene_symbol": "ADNP2"
}